{
  "gene": "UniProtKB:P42224",
  "gene_symbol": "STAT1",
  "term_id": "GO:0006952",
  "gene_name": "Signal transducer and activator of transcription 1-alpha_beta",
  "term_label": "defense response"
}